{
  "term_label": "calcium ion binding",
  "gene_name": "Calcineurin B homologous protein 1",
  "term_id": "GO:0005509",
  "gene": "UniProtKB:Q99653",
  "gene_symbol": "CHP1"
}